positive regulation of membrane repolarization during atrial cardiac muscle cell action potential [GO:1905002] (biological process) Also known as: up regulation of membrane repolarization during atrial cardiac muscle cell action potential, up-regulation of membrane repolarization during atrial cardiac muscle cell action potential, upregulation of membrane repolarization during atrial cardiac muscle cell action potential, activation of membrane repolarization during atrial cardiac muscle cell action potential, activation of atrial repolarization, activation of electrocardiogram QRS complex, positive regulation of atrial repolarization, positive regulation of electrocardiogram QRS complex, up regulation of atrial repolarization, up regulation of electrocardiogram QRS complex, up-regulation of atrial repolarization, up-regulation of electrocardiogram QRS complex, upregulation of atrial repolarization, upregulation of electrocardiogram QRS complex Definition: Any process that activates or increases the frequency, rate or extent of membrane repolarization during atrial cardiac muscle cell action potential. Relationships: is a type of regulation of membrane repolarization during atrial cardiac muscle cell action potential [GO:1905000]; is a type of GO:1905033; positively regulates membrane repolarization during atrial cardiac muscle cell action potential [GO:0098914] References: PMID:21098446 Sources: GOC:BHF, GOC:BHF_miRNA, GOC:TermGenie, GOC:mtg_cardiac_conduct_nov11, GOC:rph